positive regulation of DNA-templated transcription, elongation [GO:0032786] (biological process) Also known as: activation of RNA elongation, positive regulation of transcription elongation, positive regulation of transcriptional elongation, stimulation of RNA elongation, up regulation of RNA elongation, up-regulation of RNA elongation, upregulation of RNA elongation, positive regulation of DNA-dependent transcription, elongation, positive regulation of transcription elongation, DNA-dependent, positive transcription elongation regulator activity Relationships: is a type of regulation of DNA-templated transcription elongation [GO:0032784]; is a type of positive regulation of DNA-templated transcription [GO:0045893]; positively regulates GO:0006354 Subtypes: positive regulation of transcription elongation by RNA polymerase II [GO:0032968], GO:2001209 Sources: GOC:mah, GOC:txnOH Definition: Any process that activates or increases the frequency, rate or extent of transcription elongation, the extension of an RNA molecule after transcription initiation and promoter clearance by the addition of ribonucleotides catalyzed by a DNA-dependent RNA polymerase.